{
  "gene_symbol": "IGHV5-10-1",
  "term_id": "GO:0016064",
  "gene": "UniProtKB:A0A0J9YXX1",
  "term_label": "immunoglobulin mediated immune response",
  "gene_name": "Immunoglobulin heavy variable 5-10-1"
}